{
  "gene": "UniProtKB:Q6WQI6",
  "gene_symbol": "HEPN1",
  "gene_name": "Putative cancer susceptibility gene HEPN1 protein",
  "term_id": "UNKNOWN:0002",
  "term_label": "Unknown biological process"
}